thiocyanate peroxidase activity [GO:0036393] (molecular function) Relationships: is a type of peroxidase activity [GO:0004601]; is part of GO:0018969 Also known as: lactoperoxidase activity Definition: Catalysis of the reaction: thiocyanate (SCN-) + hydrogen peroxide (H2O2) = hypothiocyanite (OSCN-) + 2 H2O. Catalyzes the hydrogen peroxide oxidation of thiocyanate. References: PMID:12626341 Sources: GOC:pm